G-protein beta-subunit binding [GO:0031681] (molecular function) Definition: Binding to a G-protein beta subunit. Relationships: is a type of protein binding [GO:0005515] Also known as: G-beta protein subunit binding Sources: GOC:mah